EARP complex [GO:1990745] (cellular component) Relationships: is a type of GO:0032991; is part of recycling endosome [GO:0055037] Definition: A quatrefoil tethering complex required for endocytic recycling. References: PMID:25799061